negative regulation of tyramine signaling pathway [GO:2000132] (biological process) Definition: Any process that stops, prevents, or reduces the frequency, rate or extent of tyramine signaling pathway. Sources: GOC:mah Also known as: negative regulation of tyramine signalling pathway Relationships: is a type of negative regulation of octopamine or tyramine signaling pathway [GO:2000126]; is a type of GO:2000131; negatively regulates tyramine signaling pathway [GO:0071928]